{
  "gene_name": "Selenoprotein M",
  "term_label": "oxidoreductase activity",
  "term_id": "GO:0016491",
  "gene_symbol": "SELENOM",
  "gene": "UniProtKB:Q8WWX9"
}